{
  "gene_name": "TGF-beta receptor type-2",
  "term_id": "GO:0048185",
  "gene": "UniProtKB:P37173",
  "term_label": "activin binding",
  "gene_symbol": "TGFBR2"
}